pelargonidin 3-O-glucoside biosynthetic process [GO:0033487] (biological process) Sources: GOC:mah, MetaCyc:PWY-5125 Definition: The chemical reactions and pathways resulting in the formation of pelargonidin 3-O-glucoside, a basic anthocyanin responsible for red to magenta coloration of flowers and fruits. Also known as: pelargonidin 3-O-glucoside anabolism, pelargonidin 3-O-glucoside biosynthesis, pelargonidin 3-O-glucoside formation, pelargonidin 3-O-glucoside synthesis Relationships: is a type of flavonoid biosynthetic process [GO:0009813]; is_a beta-glucoside biosynthetic process [GO:1901806]